{
  "term_label": "regulation of transcription by RNA polymerase II",
  "gene": "UniProtKB:Q13461",
  "term_id": "GO:0006357",
  "gene_symbol": "FOXE3",
  "gene_name": "Forkhead box protein E3"
}